{
  "gene": "UniProtKB:P29350",
  "term_label": "non-membrane spanning protein tyrosine phosphatase activity",
  "gene_symbol": "PTPN6",
  "term_id": "GO:0004726",
  "gene_name": "Tyrosine-protein phosphatase non-receptor type 6"
}